{
  "gene": "UniProtKB:Q86X24",
  "term_id": "GO:0051598",
  "gene_name": "HORMA domain-containing protein 1",
  "gene_symbol": "HORMAD1",
  "term_label": "meiotic recombination checkpoint signaling"
}